{
  "gene": "UniProtKB:Q9UEU5",
  "term_id": "UNKNOWN:0003",
  "gene_symbol": "GAGE8",
  "term_label": "Unknown cellular component",
  "gene_name": "G antigen 2D"
}